{
  "gene": "UniProtKB:Q6VVX0",
  "gene_symbol": "CYP2R1",
  "term_id": "GO:0030343",
  "term_label": "vitamin D3 25-hydroxylase activity",
  "gene_name": "Vitamin D 25-hydroxylase"
}